{
  "gene_symbol": "C8orf89",
  "term_id": "UNKNOWN:0001",
  "gene": "UniProtKB:P0DMQ9",
  "gene_name": "Putative uncharacterized protein C8orf89",
  "term_label": "Unknown molecular function"
}